{
  "gene_name": "Transport and Golgi organization protein 1 homolog",
  "gene": "UniProtKB:Q5JRA6",
  "term_id": "GO:0035459",
  "term_label": "vesicle cargo loading",
  "gene_symbol": "MIA3"
}